DNA alpha-glucosyltransferase activity [GO:0033820] (molecular function) Definition: Catalysis of the transfer of an alpha-D-glucosyl residue from UDP-glucose to a hydroxymethylcytosine residue in DNA. Relationships: is a type of glucosyltransferase activity [GO:0046527]; is a type of catalytic activity, acting on DNA [GO:0140097] Sources: EC:2.4.1.26 Also known as: T2-HMC-alpha-glucosyl transferase activity, T4-HMC-alpha-glucosyl transferase activity, T6-HMC-alpha-glucosyl transferase activity, UDP-glucose:DNA alpha-D-glucosyltransferase activity, UDPglucose-DNA alpha-glucosyltransferase activity, uridine diphosphoglucose-deoxyribonucleate alpha-glucosyltransferase activity